{
  "gene_name": "Dopamine beta-hydroxylase",
  "gene_symbol": "DBH",
  "term_label": "norepinephrine biosynthetic process",
  "gene": "UniProtKB:P09172",
  "term_id": "GO:0042421"
}